{
  "term_id": "GO:0043277",
  "gene_symbol": "TIMD4",
  "gene_name": "T-cell immunoglobulin and mucin domain-containing protein 4",
  "term_label": "apoptotic cell clearance",
  "gene": "UniProtKB:Q96H15"
}